{
  "term_label": "respiratory electron transport chain",
  "term_id": "GO:0022904",
  "gene_symbol": "SDHB",
  "gene": "UniProtKB:P21912",
  "gene_name": "Succinate dehydrogenase [ubiquinone] iron-sulfur subunit, mitochondrial"
}